{
  "term_label": "Unknown biological process",
  "gene": "UniProtKB:Q149M9",
  "gene_symbol": "NWD1",
  "gene_name": "NACHT domain- and WD repeat-containing protein 1",
  "term_id": "UNKNOWN:0002"
}